{
  "gene": "UniProtKB:Q9H2S1",
  "term_label": "dendritic spine",
  "term_id": "GO:0043197",
  "gene_name": "Small conductance calcium-activated potassium channel protein 2",
  "gene_symbol": "KCNN2"
}